box H/ACA sno(s)RNA 3'-end processing [GO:0000495] (BP) Also known as: box H/ACA RNA 3' end processing, box H/ACA sRNA 3'-end processing, box H/ACA snoRNA 3'-end processing Definition: Any process involved in forming the mature 3' end of a box H/ACA RNA molecule. Relationships: is a type of sno(s)RNA 3'-end processing [GO:0031126]; is a type of box H/ACA sno(s)RNA processing [GO:0034964] Sources: GOC:krc